{
  "gene": "UniProtKB:Q96HE9",
  "gene_name": "Proline-rich protein 11",
  "term_id": "GO:0005737",
  "term_label": "cytoplasm",
  "gene_symbol": "PRR11"
}